{
  "gene_symbol": "UBR4",
  "term_label": "ubiquitin-dependent protein catabolic process via the N-end rule pathway",
  "term_id": "GO:0071596",
  "gene": "UniProtKB:Q5T4S7",
  "gene_name": "E3 ubiquitin-protein ligase UBR4"
}